collagen trimer [GO:0005581] (cellular component) Relationships: is a type of GO:0032991 References: PMID:19693541, PMID:21421911 Sources: GOC:dos, GOC:mah Definition: A protein complex consisting of three collagen chains assembled into a left-handed triple helix. These trimers typically assemble into higher order structures. Subtypes: GO:0005583, FACIT collagen trimer [GO:0005593], GO:0030936, network-forming collagen trimer [GO:0098642], multiplexin collagen trimer [GO:0140156], von-Willerbrand-factor-A-domain-rich collagen trimer [GO:0140158], collagen type XIX trimer [GO:1990318], collagen type XXVI trimer [GO:1990324]